regulation of IP-10 production [GO:0071658] (BP) Also known as: regulation of CXCL10 production, regulation of chemokine (C-C motif) ligand 10 production Relationships: is a type of GO:0032642; regulates IP-10 production [GO:0071612] Sources: GOC:mah Definition: Any process that modulates the frequency, rate, or extent of production of IP-10. Subtypes: negative regulation of IP-10 production [GO:0071659], positive regulation of IP-10 production [GO:0071660]